{
  "term_id": "GO:0000978",
  "gene_symbol": "PRDM15",
  "gene_name": "PR domain zinc finger protein 15",
  "gene": "UniProtKB:P57071",
  "term_label": "RNA polymerase II cis-regulatory region sequence-specific DNA binding"
}